ground tissue pattern formation [GO:1990064] (biological process) References: PMID:23444357 Also known as: ground tissue patterning Definition: The regionalization process that gives rise to the patterning of the ground tissue. Relationships: is a type of regionalization [GO:0003002]